{
  "gene_name": "Guanine nucleotide-binding protein-like 1",
  "term_label": "Unknown cellular component",
  "gene_symbol": "GNL1",
  "gene": "UniProtKB:P36915",
  "term_id": "UNKNOWN:0003"
}